{
  "term_id": "GO:0045087",
  "gene": "UniProtKB:Q86UV7",
  "term_label": "innate immune response",
  "gene_name": "Tripartite motif-containing protein 73",
  "gene_symbol": "TRIM73"
}